{
  "term_label": "olfactory receptor activity",
  "gene_symbol": "OR10G2",
  "term_id": "GO:0004984",
  "gene_name": "Olfactory receptor 10G2",
  "gene": "UniProtKB:Q8NGC3"
}